{
  "gene_symbol": "N4BP1",
  "term_label": "negative regulation of protein ubiquitination",
  "gene": "UniProtKB:O75113",
  "gene_name": "NEDD4-binding protein 1",
  "term_id": "GO:0031397"
}